{
  "gene_symbol": "CLEC18A",
  "gene_name": "C-type lectin domain family 18 member A",
  "gene": "UniProtKB:A5D8T8",
  "term_label": "extracellular space",
  "term_id": "GO:0005615"
}